{
  "gene": "UniProtKB:P48723",
  "term_id": "GO:0005886",
  "term_label": "plasma membrane",
  "gene_name": "Heat shock 70 kDa protein 13",
  "gene_symbol": "HSPA13"
}